HECT domain binding [GO:0032399] (molecular function) Definition: Binding to a HECT, 'Homologous to the E6-AP Carboxy-Terminus', domain of a protein. Relationships: is a type of GO:0019904 Sources: GOC:mah, Pfam:PF00632